ubiquinone biosynthesis complex [GO:0110142] (cellular component) Definition: A protein complex composed of enzymes and accessory factors of the ubiquinone (CoQ) biosynthesis pathway. In E. coli, the complex is composed of seven proteins: UbiE, F, G, H, I, J and K. In eukaryotes, the complex is located on the matrix face of the inner mitochondrial membrane and includes COQ3, COQ4, COQ5, COQ6, COQ7, COQ9. Relationships: is a type of catalytic complex [GO:1902494] Also known as: CoQ Biosynthetic Complex, CoQ metabolon, CoQ-synthome, Ubi complex, complex Q References: PMID:27060254, PMID:28927698, PMID:30686758 Sources: GOC:imk